regulation of DNA recombinase disassembly [GO:0062109] (biological process) References: PMID:30297419 Relationships: is a type of GO:0043244; regulates DNA recombinase disassembly [GO:1990986] Subtypes: negative regulation of DNA recombinase disassembly [GO:0062110] Definition: Any process that modulates the rate, frequency or extent of DNA recombinase disassembly, the disaggregation of a DNA recombinase complex into its constituent components.